{
  "term_id": "GO:0042391",
  "term_label": "regulation of membrane potential",
  "gene_symbol": "GRIN1",
  "gene_name": "Glutamate receptor ionotropic, NMDA 1",
  "gene": "UniProtKB:Q05586"
}